{
  "gene_name": "Dihydropyrimidinase-related protein 1",
  "gene_symbol": "CRMP1",
  "term_label": "hydrolase activity, acting on carbon-nitrogen (but not peptide) bonds, in cyclic amides",
  "gene": "UniProtKB:Q14194",
  "term_id": "GO:0016812"
}